positive regulation of B cell proliferation [GO:0030890] (biological process) Relationships: is a type of GO:0030888; is a type of GO:0050671; is a type of GO:0050871; positively regulates B cell proliferation [GO:0042100] Also known as: positive regulation of B lymphocyte proliferation, positive regulation of B-cell proliferation, positive regulation of B-lymphocyte proliferation, up regulation of B cell proliferation, up-regulation of B cell proliferation, upregulation of B cell proliferation, activation of B cell proliferation, stimulation of B cell proliferation Definition: Any process that activates or increases the rate or extent of B cell proliferation. Sources: GOC:mah